{
  "gene": "UniProtKB:P04899",
  "gene_symbol": "GNAI2",
  "gene_name": "Guanine nucleotide-binding protein G(i) subunit alpha-2",
  "term_label": "cytoplasm",
  "term_id": "GO:0005737"
}